{
  "gene_name": "Transmembrane protein 266",
  "gene": "UniProtKB:Q2M3C6",
  "term_id": "UNKNOWN:0001",
  "term_label": "Unknown molecular function",
  "gene_symbol": "TMEM266"
}